{
  "gene_name": "Transcriptional activator GLI3",
  "term_label": "RNA polymerase II cis-regulatory region sequence-specific DNA binding",
  "gene": "UniProtKB:P10071",
  "gene_symbol": "GLI3",
  "term_id": "GO:0000978"
}